{
  "term_id": "UNKNOWN:0003",
  "term_label": "Unknown cellular component",
  "gene_name": "Albumin",
  "gene_symbol": "ALB",
  "gene": "UniProtKB:P02768"
}